flavonol 3-O-arabinosyltransferase activity [GO:0080059] (molecular function) References: PMID:18757557 Relationships: is a type of GO:0008194; is a type of arabinosyltransferase activity [GO:0052636] Definition: Catalysis of the reaction: UDP-arabinose + a flavonol = UDP + a flavonol 3-O-D-arabinoside.